deoxyribonucleotide binding [GO:0032552] (MF) Definition: Binding to a deoxyribonucleotide, any compound consisting of a deoxyribonucleoside that is esterified with (ortho)phosphate or an oligophosphate at any hydroxyl group on the deoxyribose moiety. Sources: GOC:mah Subtypes: purine deoxyribonucleotide binding [GO:0032554], GO:0032556 Relationships: is a type of GO:0000166; is a type of carbohydrate derivative binding [GO:0097367]